{
  "gene_symbol": "CARMIL1",
  "term_id": "GO:0016477",
  "gene": "UniProtKB:Q5VZK9",
  "gene_name": "F-actin-uncapping protein LRRC16A",
  "term_label": "cell migration"
}